1-(3,5-dichloro-2,6-dihydroxy-4-methoxyphenyl)hexan-1-one metabolic process [GO:0031147] (biological process) Also known as: 1-(3,5-dichloro-2,6-dihydroxy-4-methoxyphenyl)hexan-1-one metabolism, DIF-1 metabolic process, DIF-1 metabolism References: PMID:10706822 Sources: GOC:mah Subtypes: DIF-1 biosynthetic process [GO:0031148] Definition: The chemical reactions and pathways involving 1-(3,5-dichloro-2,6-dihydroxy-4-methoxyphenyl)hexan-1-one, also known as DIF-1, differentiation-inducing factor-1. DIF-1 is a secreted chlorinated molecule that controls cell fate during development of Dictyostelium cells. Relationships: is a type of phenol-containing compound metabolic process [GO:0018958]; is a type of ketone metabolic process [GO:0042180]; is a type of benzene-containing compound metabolic process [GO:0042537]; is a type of organohalogen metabolic process [GO:0090345]; has part DIF dechlorinase activity [GO:0099085]